positive regulation of neuron projection arborization [GO:0150012] (biological process) Definition: Any process that activates or increases the frequency, rate or extent of the process in which the anatomical structures of a neuron projection are generated and organized into branches. Relationships: is a type of positive regulation of cell projection organization [GO:0031346]; is a type of positive regulation of developmental process [GO:0051094]; is a type of regulation of neuron projection arborization [GO:0150011]; positively regulates neuron projection arborization [GO:0140058] Also known as: positive regulation of neurite arborization, positive regulation of neurite branching, positive regulation of neuron projection branching References: PMID:17114044 Sources: GOC:aruk, GOC:bc